myoblast migration involved in skeletal muscle regeneration [GO:0014839] (BP) Definition: The process in which a myoblast migrates along an entire fiber to the site of injury. A myoblast is a mononucleate cell type that, by fusion with other myoblasts, gives rise to the myotubes that eventually develop into skeletal muscle fibers. References: PMID:16607119 Sources: CL:0000056, GOC:ef, GOC:mtg_muscle Also known as: mononucleate cell migration involved in skeletal muscle regeneration Relationships: is a type of GO:0051451; is part of skeletal muscle tissue regeneration [GO:0043403]